{
  "term_label": "nuclear pore central transport channel",
  "gene": "UniProtKB:Q9NPJ8",
  "gene_symbol": "NXT2",
  "gene_name": "NTF2-related export protein 2",
  "term_id": "GO:0044613"
}